{
  "term_id": "GO:0005634",
  "gene": "UniProtKB:Q13362",
  "term_label": "nucleus",
  "gene_name": "Serine_threonine-protein phosphatase 2A 56 kDa regulatory subunit gamma isoform",
  "gene_symbol": "PPP2R5C"
}